{
  "term_label": "Unknown cellular component",
  "gene_name": "Immunoglobulin heavy variable 3-30",
  "term_id": "UNKNOWN:0003",
  "gene": "UniProtKB:P01768",
  "gene_symbol": "IGHV3-30"
}